{
  "gene_symbol": "SPACA3",
  "gene_name": "Sperm acrosome membrane-associated protein 3",
  "gene": "UniProtKB:Q8IXA5",
  "term_label": "acrosomal vesicle",
  "term_id": "GO:0001669"
}